MLL3/4 complex [GO:0044666] (cellular component) Definition: A protein complex that can methylate lysine-4 of histone H3, and which contains either of the protein subunits MLL3 or MLL4 in mammals, or equivalent in other species. Also known as: Trr/COMPASS-like complex Relationships: is_a GO:0035097 References: PMID:21875999 Sources: GOC:sart